deoxyribonucleoside catabolic process [GO:0046121] (BP) Also known as: deoxyribonucleoside breakdown, deoxyribonucleoside catabolism, deoxyribonucleoside degradation Subtypes: purine deoxyribonucleoside catabolic process [GO:0046124], pyrimidine deoxyribonucleoside catabolic process [GO:0046127] Relationships: is a type of deoxyribonucleoside metabolic process [GO:0009120]; is a type of nucleoside catabolic process [GO:0009164] Sources: GOC:ai Definition: The chemical reactions and pathways resulting in the breakdown of any one of a family of organic molecules consisting of a purine or pyrimidine base covalently bonded to a sugar deoxyribose (a deoxyribonucleoside).